{
  "gene_symbol": "DHRSX",
  "term_id": "GO:0010508",
  "gene_name": "Dehydrogenase_reductase SDR family member on chromosome X",
  "gene": "UniProtKB:Q8N5I4",
  "term_label": "positive regulation of autophagy"
}